regulation of actomyosin structure organization [GO:0110020] (biological process) Definition: Any process that modulates the frequency, rate or extent of the assembly, arrangement of constituent parts, or disassembly of cytoskeletal structures containing both actin and myosin or paramyosin. Relationships: is a type of regulation of actin cytoskeleton organization [GO:0032956]; regulates actomyosin structure organization [GO:0031032] Subtypes: regulation of stress fiber assembly [GO:0051492], GO:0060297, GO:1905304, GO:2000431 References: PMID:22790195 Sources: GOC:lf